{
  "gene_symbol": "EMC8",
  "gene": "UniProtKB:O43402",
  "term_id": "GO:0071816",
  "gene_name": "ER membrane protein complex subunit 8",
  "term_label": "tail-anchored membrane protein insertion into ER membrane"
}